{
  "term_label": "response to exogenous dsRNA",
  "gene": "UniProtKB:P01566",
  "term_id": "GO:0043330",
  "gene_name": "Interferon alpha-10",
  "gene_symbol": "IFNA10"
}